{
  "term_id": "GO:0045121",
  "gene": "UniProtKB:P04156",
  "gene_name": "Major prion protein",
  "term_label": "membrane raft",
  "gene_symbol": "PRNP"
}